{
  "term_id": "GO:0007015",
  "gene_symbol": "LMOD1",
  "term_label": "actin filament organization",
  "gene_name": "Leiomodin-1",
  "gene": "UniProtKB:P29536"
}